{
  "gene_symbol": "HORMAD2",
  "gene": "UniProtKB:Q8N7B1",
  "term_id": "GO:0007130",
  "gene_name": "HORMA domain-containing protein 2",
  "term_label": "synaptonemal complex assembly"
}